{
  "term_id": "UNKNOWN:0003",
  "gene": "UniProtKB:A8MUU9",
  "gene_symbol": "A8MUU9",
  "gene_name": "Putative uncharacterized protein ENSP00000383309",
  "term_label": "Unknown cellular component"
}